regulation of presynaptic membrane potential [GO:0099505] (biological process) Also known as: regulation of pre-synaptic membrane potential Sources: GOC:dph, GOC:ef Relationships: is a type of regulation of membrane potential [GO:0042391] Definition: Any process that modulates the potential difference across a presynaptic membrane.